{
  "gene_name": "DNA-3-methyladenine glycosylase",
  "gene_symbol": "MPG",
  "term_id": "GO:0003905",
  "gene": "UniProtKB:P29372",
  "term_label": "alkylbase DNA N-glycosylase activity"
}